{
  "gene": "UniProtKB:Q92542",
  "gene_name": "Nicastrin",
  "term_label": "Notch receptor processing",
  "gene_symbol": "NCSTN",
  "term_id": "GO:0007220"
}